asparagine synthase (glutamine-hydrolyzing) activity [GO:0004066] (molecular function) Also known as: AS, AS-B activity, L-aspartate:L-glutamine amido-ligase (AMP-forming), asparagine synthase (glutamine-hydrolysing), asparagine synthetase (glutamine-hydrolysing), asparagine synthetase (glutamine-hydrolyzing) activity, asparagine synthetase B activity, glutamine-dependent asparagine synthetase activity Sources: EC:6.3.5.4, RHEA:12228 Definition: Catalysis of the reaction: ATP + L-aspartate + L-glutamine = AMP + diphosphate + L-asparagine + L-glutamate. Relationships: is_a GO:0016884